prevention of polyspermy during double fertilization [GO:0160071] (BP) References: PMID:27951463 Definition: The regulation of double fertilization forming a zygote and endosperm process that ensures that only a single sperm cell fertilizes one egg cell and another single sperm cell fertilizes one central cell. Relationships: is a type of GO:0080155